{
  "gene_symbol": "DZIP3",
  "term_id": "GO:0031593",
  "term_label": "polyubiquitin modification-dependent protein binding",
  "gene": "UniProtKB:Q86Y13",
  "gene_name": "E3 ubiquitin-protein ligase DZIP3"
}